{
  "gene": "UniProtKB:P03905",
  "term_label": "ubiquinone binding",
  "gene_symbol": "MT-ND4",
  "term_id": "GO:0048039",
  "gene_name": "NADH-ubiquinone oxidoreductase chain 4"
}